cell growth mode switching, budding to filamentous [GO:0036187] (biological process) Also known as: yeast to hyphal transition Sources: GOC:di Definition: The process in which a cell switches from growing as a round budding cell to growing as a filament (elongated cells attached end-to-end). An example of this is the yeast-hyphal transition of Candida albicans. Relationships: is_a regulation of growth of unicellular organism as a thread of attached cells [GO:0070784]